regulation of phosphatidylinositol dephosphorylation [GO:0060304] (biological process) Relationships: is a type of regulation of dephosphorylation [GO:0035303]; is a type of regulation of macromolecule metabolic process [GO:0060255]; is_a regulation of phospholipid metabolic process [GO:1903725]; regulates phosphatidylinositol dephosphorylation [GO:0046856] Sources: GOC:dph, GOC:tb Definition: Any process that modulates the frequency, rate or extent of the chemical reaction involving the removal of one or more phosphate groups from a phosphatidylinositol. Also known as: regulation of phosphoinositide dephosphorylation